{
  "term_id": "GO:0007029",
  "gene_name": "Protein transport protein Sec16A",
  "gene_symbol": "SEC16A",
  "gene": "UniProtKB:O15027",
  "term_label": "endoplasmic reticulum organization"
}